{
  "gene_symbol": "RARS1",
  "gene": "UniProtKB:P54136",
  "term_label": "Unknown cellular component",
  "term_id": "UNKNOWN:0003",
  "gene_name": "Arginine--tRNA ligase, cytoplasmic"
}